{
  "gene": "UniProtKB:Q8WZA6",
  "term_id": "GO:0004984",
  "term_label": "olfactory receptor activity",
  "gene_symbol": "OR1E3",
  "gene_name": "Olfactory receptor 1E3"
}